(+)-secoisolariciresinol monoglucoside glucosyltransferase activity [GO:0102611] (molecular function) Definition: Catalysis of the reaction: (+)-secoisolariciresinol monoglucoside + UDP-alpha-D-glucose = (+)-secoisolariciresinol diglucoside + UDP + H+. Relationships: is a type of GO:0016758 References: PMID:24678929 Sources: GOC:pz